regulation of protein depolymerization [GO:1901879] (biological process) Subtypes: GO:0030834, regulation of intermediate filament depolymerization [GO:0030842], regulation of microtubule depolymerization [GO:0031114], regulation of COPII vesicle uncoating [GO:0090111], GO:1901880, positive regulation of protein depolymerization [GO:1901881], regulation of synaptic vesicle uncoating [GO:1903388] Definition: Any process that modulates the frequency, rate or extent of protein depolymerization. Relationships: is a type of regulation of protein-containing complex disassembly [GO:0043244]; regulates protein depolymerization [GO:0051261] Also known as: regulation of protein polymer breakdown, regulation of protein polymer catabolic process, regulation of protein polymer catabolism, regulation of protein polymer degradation References: PMID:12032137 Sources: GOC:BHF, GOC:TermGenie, GOC:rl